{
  "term_id": "GO:0005886",
  "gene": "UniProtKB:Q8NCK7",
  "gene_symbol": "SLC16A11",
  "term_label": "plasma membrane",
  "gene_name": "Monocarboxylate transporter 11"
}